{
  "term_label": "replication fork",
  "gene_name": "DNA repair protein XRCC3",
  "term_id": "GO:0005657",
  "gene_symbol": "XRCC3",
  "gene": "UniProtKB:O43542"
}